{
  "gene_name": "[Pyruvate dehydrogenase (acetyl-transferring)] kinase isozyme 2, mitochondrial",
  "term_id": "GO:0004740",
  "gene": "UniProtKB:Q15119",
  "gene_symbol": "PDK2",
  "term_label": "pyruvate dehydrogenase (acetyl-transferring) kinase activity"
}